{
  "term_label": "Unknown biological process",
  "gene_name": "F-box only protein 40",
  "term_id": "UNKNOWN:0002",
  "gene": "UniProtKB:Q9UH90",
  "gene_symbol": "FBXO40"
}